{
  "gene": "UniProtKB:Q49AJ0",
  "term_label": "Unknown cellular component",
  "gene_name": "Protein FAM135B",
  "gene_symbol": "FAM135B",
  "term_id": "UNKNOWN:0003"
}